alcohol O-acyltransferase activity [GO:0034318] (molecular function) Definition: Catalysis of the transfer of an acyl group to an oxygen atom on an alcohol acceptor molecule. Subtypes: alcohol O-acetyltransferase activity [GO:0004026] Relationships: is_a O-acyltransferase activity [GO:0008374] Sources: GOC:mah Also known as: acyl-CoA:alcohol O-acyltransferase activity, acyl-coenzymeA:alcohol O-acyltransferase activity, alcohol acyltransferase activity, AEATase activity, acyl-CoA:ethanol O-acyltransferase, acyl-coenzymeA:ethanol O-acyltransferase activity